cohesin unloader activity [GO:0140670] (molecular function) Also known as: cohesin unloading activity Definition: Facilitating a conformational change to unload a cohesin complex from sister chromatids. Relationships: is a type of GO:0140097 References: PMID:26687354